{
  "term_label": "Unknown molecular function",
  "term_id": "UNKNOWN:0001",
  "gene_symbol": "CYSTM1",
  "gene": "UniProtKB:Q9H1C7",
  "gene_name": "Cysteine-rich and transmembrane domain-containing protein 1"
}